perichondral bone morphogenesis [GO:0061974] (biological process) Relationships: is a type of GO:0061973 Definition: The process in which bones are generated and organized as a result of the conversion of initial connective tissue surrounding cartilage into bone. References: PMID:21901110